mesenchymal cell differentiation involved in bone development [GO:1901706] (BP) Definition: The process in which relatively unspecialized cells acquire specialized structural and/or functional features that characterize the mesenchymal cells of bone as it progresses from its formation to the mature state. References: PMID:21571217 Sources: GOC:TermGenie, GOC:hjd Relationships: is a type of mesenchymal cell differentiation [GO:0048762]; is part of bone development [GO:0060348]